{
  "term_label": "protein serine/threonine kinase activity",
  "gene_symbol": "OXSR1",
  "term_id": "GO:0004674",
  "gene_name": "Serine_threonine-protein kinase OSR1",
  "gene": "UniProtKB:O95747"
}